{
  "term_id": "UNKNOWN:0002",
  "gene_name": "Coiled-coil domain-containing protein 30",
  "gene_symbol": "CCDC30",
  "gene": "UniProtKB:Q5VVM6",
  "term_label": "Unknown biological process"
}